apigenin-7,4'-dimethyl ether 6-hydroxylase activity [GO:0102534] (molecular function) Sources: RHEA:73435 Definition: Catalysis of the reaction: apigenin 4',7-dimethyl ether + O2 + reduced [NADPH--hemoprotein reductase] = H+ + H2O + ladanein + oxidized [NADPH--hemoprotein reductase]. Relationships: is a type of oxidoreductase activity, acting on paired donors, with incorporation or reduction of molecular oxygen, NAD(P)H as one donor, and incorporation of one atom of oxygen [GO:0016709]